{
  "term_label": "cytosol",
  "gene": "UniProtKB:Q9H347",
  "term_id": "GO:0005829",
  "gene_name": "Ubiquilin-3",
  "gene_symbol": "UBQLN3"
}